progesterone 21-hydroxylase activity [GO:0106309] (molecular function) Relationships: is a type of steroid 21-monooxygenase activity [GO:0004509] References: PMID:25855791 Sources: RHEA:50304 Definition: Catalysis of the reaction: O2 + progesterone + reduced [NADPH--hemoprotein reductase] = 21-hydroxyprogesterone + H+ + H2O + oxidized [NADPH--hemoprotein reductase].